{
  "gene": "UniProtKB:A8MXV4",
  "term_label": "Unknown molecular function",
  "gene_symbol": "NUDT19",
  "gene_name": "Acyl-coenzyme A diphosphatase NUDT19",
  "term_id": "UNKNOWN:0001"
}